{
  "gene_symbol": "OR51B4",
  "term_label": "olfactory receptor activity",
  "gene": "UniProtKB:Q9Y5P0",
  "gene_name": "Olfactory receptor 51B4",
  "term_id": "GO:0004984"
}